regulation of mitochondrial RNA catabolic process [GO:0000960] (BP) Subtypes: negative regulation of mitochondrial RNA catabolic process [GO:0000961], positive regulation of mitochondrial RNA catabolic process [GO:0000962], regulation of mitochondrial mRNA catabolic process [GO:1905637] Definition: Any process that modulates the frequency, rate or extent of the chemical reactions and pathways involving catabolism in the mitochondrion of RNA transcribed from the mitochondrial genome. Sources: GOC:krc, GOC:mah Relationships: is_a regulation of catabolic process [GO:0009894]; is a type of regulation of RNA metabolic process [GO:0051252]; regulates GO:0000957